{
  "gene_symbol": "JAM2",
  "term_label": "Unknown molecular function",
  "gene_name": "Junctional adhesion molecule B",
  "gene": "UniProtKB:P57087",
  "term_id": "UNKNOWN:0001"
}